{
  "term_id": "UNKNOWN:0001",
  "term_label": "Unknown molecular function",
  "gene": "UniProtKB:Q96M83",
  "gene_symbol": "CCDC7",
  "gene_name": "Coiled-coil domain-containing protein 7"
}